{
  "term_label": "Unknown molecular function",
  "gene": "UniProtKB:Q9BS92",
  "gene_name": "Protein NipSnap homolog 3B",
  "term_id": "UNKNOWN:0001",
  "gene_symbol": "NIPSNAP3B"
}